{
  "gene": "UniProtKB:P02649",
  "gene_symbol": "APOE",
  "term_label": "very-low-density lipoprotein particle",
  "gene_name": "Apolipoprotein E",
  "term_id": "GO:0034361"
}